{
  "gene": "UniProtKB:Q7L5Y1",
  "term_label": "hydro-lyase activity",
  "gene_name": "Mitochondrial enolase superfamily member 1",
  "term_id": "GO:0016836",
  "gene_symbol": "ENOSF1"
}